uridine to cytidine editing [GO:0016555] (biological process) Definition: The conversion of a uridine residue to cytosine in an RNA molecule by amination. Relationships: is a type of base conversion or substitution editing [GO:0016553] References: PMID:11092837